glucuronate-2-sulfatase activity [GO:0015024] (molecular function) Also known as: glucuronate-2-sulphatase activity, chondro-2-sulfatase activity, glucurono-2-sulfatase activity, polysaccharide-2-O-sulfo-D-glucuronate 2-sulfohydrolase activity Sources: EC:3.1.6.18 Definition: Catalysis of the hydrolysis of the 2-sulfate groups of the 2-O-sulfo-D-glucuronate residues of chondroitin sulfate, heparin and heparitin sulfate. Relationships: is a type of sulfuric ester hydrolase activity [GO:0008484]